{
  "gene_name": "Dynein axonemal heavy chain 5",
  "gene": "UniProtKB:Q8TE73",
  "term_id": "GO:0036158",
  "term_label": "outer dynein arm assembly",
  "gene_symbol": "DNAH5"
}